{
  "gene": "UniProtKB:Q13610",
  "term_id": "GO:0005634",
  "term_label": "nucleus",
  "gene_symbol": "PWP1",
  "gene_name": "Periodic tryptophan protein 1 homolog"
}